{
  "gene_name": "Polyadenylate-binding protein 2",
  "term_id": "UNKNOWN:0002",
  "term_label": "Unknown biological process",
  "gene_symbol": "PABPN1",
  "gene": "UniProtKB:Q86U42"
}